{
  "term_label": "regulation of cell projection organization",
  "term_id": "GO:0031344",
  "gene_name": "Arf-GAP with Rho-GAP domain, ANK repeat and PH domain-containing protein 1",
  "gene": "UniProtKB:Q96P48",
  "gene_symbol": "ARAP1"
}